tRNA-2-methylthio-N(6)-dimethylallyladenosine(37) synthase activity [GO:0035597] (molecular function) References: PMID:20472640 Sources: RHEA:37067 Definition: Catalysis of the reaction: N(6)-dimethylallyladenosine(37) in tRNA + [sulfur carrier]-SH + AH2 + 2 S-adenosyl-L-methionine = 2-methylsulfanyl-N(6)-dimethylallyladenosine(37) in tRNA + [sulfur carrier]-H + 5'-deoxyadenosine + L-methionine + A + S-adenosyl-L-homocysteine + 2 H+. Also known as: N6-isopentenyladenosine methylthiotransferase activity, i6A methylthiotransferase activity, tRNA-2-methylthio-N(6)-dimethylallyladenosine synthase activity Relationships: is_a methylthiotransferase activity [GO:0035596]; is a type of catalytic activity, acting on a tRNA [GO:0140101]; is part of tRNA methylthiolation [GO:0035600]